{
  "term_id": "GO:0003682",
  "term_label": "chromatin binding",
  "gene_symbol": "NAP1L3",
  "gene": "UniProtKB:Q99457",
  "gene_name": "Nucleosome assembly protein 1-like 3"
}